{
  "gene_name": "T cell receptor beta joining 1-5",
  "gene_symbol": "TRBJ1-5",
  "gene": "UniProtKB:A0A0J9YXM7",
  "term_id": "UNKNOWN:0002",
  "term_label": "Unknown biological process"
}